{
  "term_id": "GO:0005737",
  "gene": "UniProtKB:O15519",
  "gene_symbol": "CFLAR",
  "term_label": "cytoplasm",
  "gene_name": "CASP8 and FADD-like apoptosis regulator"
}